{
  "term_label": "negative regulation of bone mineralization involved in bone maturation",
  "gene_symbol": "RFLNA",
  "gene": "UniProtKB:Q6ZTI6",
  "gene_name": "Refilin-A",
  "term_id": "GO:1900158"
}